{
  "gene_symbol": "USP46",
  "term_label": "nucleus",
  "gene_name": "Ubiquitin carboxyl-terminal hydrolase 46",
  "term_id": "GO:0005634",
  "gene": "UniProtKB:P62068"
}